{
  "term_label": "monooxygenase activity",
  "term_id": "GO:0004497",
  "gene": "UniProtKB:Q9NR63",
  "gene_name": "Cytochrome P450 26B1",
  "gene_symbol": "CYP26B1"
}